{
  "gene": "UniProtKB:P0DPD6",
  "term_id": "GO:0005886",
  "term_label": "plasma membrane",
  "gene_name": "Endothelin-converting enzyme 2",
  "gene_symbol": "ECE2"
}